{
  "term_label": "Unknown cellular component",
  "gene_symbol": "MINDY3",
  "gene_name": "Ubiquitin carboxyl-terminal hydrolase MINDY-3",
  "term_id": "UNKNOWN:0003",
  "gene": "UniProtKB:Q9H8M7"
}